{
  "gene_symbol": "KCNA6",
  "gene": "UniProtKB:P17658",
  "gene_name": "Potassium voltage-gated channel subfamily A member 6",
  "term_label": "action potential",
  "term_id": "GO:0001508"
}